{
  "term_label": "transcription coactivator activity",
  "gene": "UniProtKB:Q92539",
  "gene_symbol": "LPIN2",
  "term_id": "GO:0003713",
  "gene_name": "Phosphatidate phosphatase LPIN2"
}